{
  "gene_name": "LIM homeobox transcription factor 1-beta",
  "term_id": "GO:0000981",
  "gene": "UniProtKB:O60663",
  "gene_symbol": "LMX1B",
  "term_label": "DNA-binding transcription factor activity, RNA polymerase II-specific"
}